positive regulation of netrin-activated signaling pathway [GO:1902843] (biological process) Also known as: positive regulation of netrin signaling pathway, positive regulation of netrin-activated signal transduction pathway, positive regulation of netrin-activated signalling pathway, positive regulation of netrin-mediated signaling pathway, up regulation of netrin signaling pathway, up regulation of netrin-activated signal transduction pathway, up regulation of netrin-activated signaling pathway, up regulation of netrin-activated signalling pathway, up regulation of netrin-mediated signaling pathway, up-regulation of netrin signaling pathway, up-regulation of netrin-activated signal transduction pathway, up-regulation of netrin-activated signaling pathway, up-regulation of netrin-activated signalling pathway, up-regulation of netrin-mediated signaling pathway, upregulation of netrin signaling pathway, upregulation of netrin-activated signal transduction pathway, upregulation of netrin-activated signaling pathway, upregulation of netrin-activated signalling pathway, upregulation of netrin-mediated signaling pathway, activation of netrin signaling pathway, activation of netrin-activated signal transduction pathway, activation of netrin-activated signaling pathway, activation of netrin-activated signalling pathway, activation of netrin-mediated signaling pathway Definition: Any process that activates or increases the frequency, rate or extent of netrin-activated signaling pathway. Relationships: is a type of GO:0009967; is a type of regulation of netrin-activated signaling pathway [GO:1902841]; positively regulates GO:0038007 References: PMID:24004945 Sources: GOC:TermGenie, GOC:kmv, GO_REF:0000058